{
  "term_id": "UNKNOWN:0003",
  "gene": "UniProtKB:Q8IWY8",
  "gene_symbol": "ZSCAN29",
  "term_label": "Unknown cellular component",
  "gene_name": "Zinc finger and SCAN domain-containing protein 29"
}